potassium:proton exchanging ATPase complex [GO:0005889] (cellular component) References: PMID:11756431 Definition: A protein complex that possesses hydrogen:potassium-exchanging ATPase activity; characterized in animal cells, where it maintains ionic gradients of K+ at the expense of ATP hydrolysis; The complex contains two obligatory subunits, the catalytic alpha subunit and a glycosylated beta subunit; two additional subunits, gamma and channel-inducing factor (CHIF), may also be present. Also known as: proton pump, hydrogen/potassium-exchanging ATPase complex, hydrogen:potassium-exchanging ATPase complex Relationships: is a type of cation-transporting ATPase complex [GO:0090533]; is a type of GO:0098797